regulation of RNA export from nucleus [GO:0046831] (biological process) Also known as: regulation of RNA export from cell nucleus, regulation of RNA export out of nucleus, regulation of RNA transport from nucleus to cytoplasm, regulation of RNA-nucleus export Definition: Any process that modulates the frequency, rate or extent of the directed movement of RNA from the nucleus to the cytoplasm. Sources: GOC:bf Subtypes: GO:0010793, negative regulation of RNA export from nucleus [GO:0046832], positive regulation of RNA export from nucleus [GO:0046833], regulation of tRNA export from nucleus [GO:2000238] Relationships: is a type of regulation of nucleobase-containing compound transport [GO:0032239]; is a type of regulation of nucleocytoplasmic transport [GO:0046822]; regulates RNA export from nucleus [GO:0006405]